{
  "term_label": "Unknown cellular component",
  "term_id": "UNKNOWN:0003",
  "gene": "UniProtKB:A8MVW0",
  "gene_name": "Protein FAM171A2",
  "gene_symbol": "FAM171A2"
}